negative regulation of cell chemotaxis to fibroblast growth factor [GO:1904848] (biological process) Subtypes: GO:2000545 Definition: Any process that stops, prevents or reduces the frequency, rate or extent of cell chemotaxis to fibroblast growth factor. References: PMID:23233752 Sources: GOC:BHF, GOC:BHF_miRNA, GOC:TermGenie, GOC:rph, GO_REF:0000058 Relationships: is a type of GO:0030336; is a type of GO:0050922; is a type of negative regulation of cellular response to growth factor stimulus [GO:0090288]; is a type of regulation of cell chemotaxis to fibroblast growth factor [GO:1904847]; negatively regulates GO:0035766 Also known as: down regulation of cell chemotaxis to fibroblast growth factor, down-regulation of cell chemotaxis to fibroblast growth factor, downregulation of cell chemotaxis to fibroblast growth factor, inhibition of cell chemotaxis to fibroblast growth factor